{
  "term_label": "calcium ion binding",
  "gene_symbol": "PLA2G2D",
  "gene": "UniProtKB:Q9UNK4",
  "gene_name": "Group IID secretory phospholipase A2",
  "term_id": "GO:0005509"
}